{
  "gene_symbol": "PADI4",
  "term_id": "GO:0005634",
  "gene": "UniProtKB:Q9UM07",
  "term_label": "nucleus",
  "gene_name": "Protein-arginine deiminase type-4"
}